{
  "gene_name": "Glypican-6",
  "term_id": "GO:0016477",
  "gene_symbol": "GPC6",
  "term_label": "cell migration",
  "gene": "UniProtKB:Q9Y625"
}